{
  "term_id": "GO:0007168",
  "gene_symbol": "GUCY2C",
  "gene_name": "Guanylyl cyclase C",
  "term_label": "receptor guanylyl cyclase signaling pathway",
  "gene": "UniProtKB:P25092"
}